retinoic acid-responsive element binding [GO:0044323] (molecular function) References: PMID:11327309, PMID:19917671 Sources: GOC:jl, GOC:vw, GOC:yaf Also known as: RARE binding Definition: Binding to a retinoic acid-responsive element, a variable direct repeat of the sequence PuGGTCA spaced by five nucleotides (DR5) found in the promoters of retinoic acid-responsive genes, to which retinoic acid receptors bind. Relationships: is a type of RNA polymerase II cis-regulatory region sequence-specific DNA binding [GO:0000978]